sweat gland development [GO:0060792] (biological process) Relationships: is a type of gland development [GO:0048732] Definition: The progression of the sweat gland over time, from its formation to the mature structure. Sweat glands secrete an aqueous solution that is used in thermoregulation. Sources: GOC:dph, GOC:sdb_2009, GOC:tb